{
  "gene": "UniProtKB:O00483",
  "gene_symbol": "NDUFA4",
  "term_label": "Unknown molecular function",
  "term_id": "UNKNOWN:0001",
  "gene_name": "Cytochrome c oxidase subunit NDUFA4"
}